maintenance of diapause [GO:0071982] (biological process) Relationships: is a type of GO:0022611 Subtypes: GO:0043055, GO:0071984 Definition: The dormancy process that results an organism remaining in diapause. Diapause is a neurohormonally mediated, dynamic state of low metabolic activity. Associated characteristics of this form of dormancy include reduced morphogenesis, increased resistance to environmental extremes, and altered or reduced behavioral activity. Full expression develops in a species-specific manner, usually in response to a number of environmental stimuli that precede unfavorable conditions. Once diapause has begun, metabolic activity is suppressed even if conditions favorable for development prevail. Once initiated, only certain stimuli are capable of releasing the organism from this state, and this characteristic is essential in distinguishing diapause from hibernation. Sources: GOC:mah